{
  "gene_name": "Nucleolar complex protein 2 homolog",
  "term_label": "Noc1p-Noc2p complex",
  "term_id": "GO:0030690",
  "gene_symbol": "NOC2L",
  "gene": "UniProtKB:Q9Y3T9"
}